{
  "gene": "UniProtKB:Q460N5",
  "gene_name": "Protein mono-ADP-ribosyltransferase PARP14",
  "term_label": "negative regulation of gene expression",
  "gene_symbol": "PARP14",
  "term_id": "GO:0010629"
}